JNK cascade [GO:0007254] (biological process) Definition: A MAPK cascade containing at least the JNK (MAPK8) MAP kinase. It starts with the activation of JUN3K (a MAPK3K), which activates JNKK a MAP2K), which in turn activates JNK. The cascade can also contain an additional tier: the upstream MAP4K. The kinases in each tier phosphorylate and activate the kinases in the downstream tier. The JNK cascade is activated by stress signals, as well as by G protein-coupled receptors, growth factors, and cytokines, and results in cellular responses such as cell proliferation, cell differentiation, apoptosis and inflammation. Relationships: is a type of MAPK cascade [GO:0000165] Regulation: regulated by GO:0046328; negatively regulated by GO:0046329; positively regulated by positive regulation of JNK cascade [GO:0046330] Also known as: SAPK cascade, stress-activated protein kinase cascade, MAPK8 cascade, c-Jun N-terminal kinase cascade, JNK1 cascade, JNK2 cascade, JNK3 cascade, MAPK10 cascade, MAPK9 cascade References: PMID:11790549, PMID:20811974, PMID:23125017